{
  "gene": "UniProtKB:Q9GZW8",
  "term_id": "GO:0007166",
  "term_label": "cell surface receptor signaling pathway",
  "gene_name": "Membrane-spanning 4-domains subfamily A member 7",
  "gene_symbol": "MS4A7"
}